hypoxanthine oxidase activity [GO:0070675] (molecular function) Definition: Catalysis of the reaction: hypoxanthine + H2O + O2 = xanthine + H2O2. Sources: GOC:mah, GOC:pde Also known as: hypoxanthine-xanthine oxidase activity, xanthine oxidoreductase activity, Schardinger enzyme activity, hypoxanthine:O2 oxidoreductase activity, hypoxanthine:oxygen oxidoreductase activity, schardinger enzyme Relationships: is a type of oxidoreductase activity, acting on CH or CH2 groups, oxygen as acceptor [GO:0016727]